{
  "term_label": "Unknown molecular function",
  "gene": "UniProtKB:Q8IYI6",
  "gene_name": "Exocyst complex component 8",
  "term_id": "UNKNOWN:0001",
  "gene_symbol": "EXOC8"
}